vitexin 2''-O-rhamnoside 7-O-methyltransferase activity [GO:0033801] (molecular function) Also known as: S-adenosyl-L-methionine:vitexin-2''-O-beta-L-rhamnoside 7-O-methyltransferase activity Definition: Catalysis of the reaction: S-adenosyl-L-methionine + vitexin 2''-O-beta-L-rhamnoside = S-adenosyl-L-homocysteine + 7-O-methylvitexin 2''-O-beta-L-rhamnoside. Sources: EC:2.1.1.153 Relationships: is a type of O-methyltransferase activity [GO:0008171]; is a type of S-adenosylmethionine-dependent methyltransferase activity [GO:0008757]